{
  "term_id": "GO:0031175",
  "term_label": "neuron projection development",
  "gene_name": "Tenascin-X",
  "gene_symbol": "TNXB",
  "gene": "UniProtKB:P22105"
}